beta-1,3-galactosyl-O-glycosyl-glycoprotein beta-1,6-N-acetylglucosaminyltransferase activity [GO:0003829] (molecular function) Definition: Catalysis of the reaction: UDP-N-acetyl-D-glucosamine + beta-D-galactosyl-(1->3)-N-acetyl-D-galactosaminyl-R = UDP + beta-D-galactosyl-(1->3)-[N-acetyl-beta-D-glucosaminyl-(1->6)]-N-acetyl-D-galactosaminyl-R. This reaction is the addition of N-acetyl-alpha-D-glucosamine to the core 1 structure of O-glycans forming core 2. Relationships: is a type of GO:0008375; is a type of catalytic activity, acting on a glycoprotein [GO:0140103] Also known as: O-glycosyl-oligosaccharide-glycoprotein N-acetylglucosaminyltransferase I activity, UDP-N-acetyl-D-glucosamine:O-glycosyl-glycoprotein (N-acetyl-D-glucosamine to N-acetyl-D-galactosamine of beta-D-galactosyl-1,3-N-acetyl-D-galactosaminyl-R) beta-1,6-N-acetyl-D-glucosaminyltransferase activity, beta(6)-N-acetylglucosaminyltransferase activity, beta6-N-acetylglucosaminyltransferase activity, core 2 acetylglucosaminyltransferase activity, core 6-beta-GlcNAc-transferase A, uridine diphosphoacetylglucosamine-mucin beta-(1,6)-acetylglucosaminyltransferase activity, uridine diphosphoacetylglucosamine-mucin beta-(1->6)-acetylglucosaminyltransferase activity Sources: EC:2.4.1.102